putrescine biosynthetic process from arginine via N-carbamoylputrescine [GO:0033390] (biological process) Also known as: putrescine anabolism from arginine via N-carbamoylputrescine, putrescine biosynthesis from arginine via N-carbamoylputrescine, putrescine formation from arginine via N-carbamoylputrescine, putrescine synthesis from arginine via N-carbamoylputrescine Sources: GOC:mah, MetaCyc:PWY-43 Relationships: is a type of putrescine biosynthetic process from arginine [GO:0033388] Definition: The chemical reactions and pathways resulting in the formation of putrescine, 1,4-diaminobutane, from other compounds, including arginine, via the intermediate N-carbamoylputrescine; in this pathway, arginine is converted to agmatine, and agmatine is converted to putrescine in two single enzymatic steps.